{
  "gene": "UniProtKB:P30939",
  "gene_name": "5-hydroxytryptamine receptor 1F",
  "gene_symbol": "HTR1F",
  "term_id": "GO:0007187",
  "term_label": "G protein-coupled receptor signaling pathway, coupled to cyclic nucleotide second messenger"
}